{
  "gene": "UniProtKB:Q8N5N7",
  "gene_name": "Large ribosomal subunit protein mL50",
  "term_id": "UNKNOWN:0001",
  "gene_symbol": "MRPL50",
  "term_label": "Unknown molecular function"
}